{
  "gene_symbol": "DLC1",
  "term_id": "GO:0035023",
  "term_label": "regulation of Rho protein signal transduction",
  "gene": "UniProtKB:Q96QB1",
  "gene_name": "Rho GTPase-activating protein 7"
}